{
  "gene": "UniProtKB:Q8NFJ8",
  "gene_name": "Class E basic helix-loop-helix protein 22",
  "gene_symbol": "BHLHE22",
  "term_label": "axon development",
  "term_id": "GO:0061564"
}